{
  "term_label": "axoneme assembly",
  "gene_name": "Radial spoke head 1 homolog",
  "gene_symbol": "RSPH1",
  "gene": "UniProtKB:Q8WYR4",
  "term_id": "GO:0035082"
}